{
  "gene_symbol": "ARMCX6",
  "term_id": "UNKNOWN:0001",
  "gene": "UniProtKB:Q7L4S7",
  "gene_name": "Protein ARMCX6",
  "term_label": "Unknown molecular function"
}